{
  "gene": "UniProtKB:Q99879",
  "term_id": "GO:0005615",
  "term_label": "extracellular space",
  "gene_symbol": "H2BC14",
  "gene_name": "Histone H2B type 1-M"
}